{
  "gene_name": "RanBP-type and C3HC4-type zinc finger-containing protein 1",
  "gene_symbol": "RBCK1",
  "term_id": "GO:0071797",
  "gene": "UniProtKB:Q9BYM8",
  "term_label": "LUBAC complex"
}